{
  "gene_symbol": "INTS7",
  "term_label": "integrator complex",
  "gene_name": "Integrator complex subunit 7",
  "gene": "UniProtKB:Q9NVH2",
  "term_id": "GO:0032039"
}